{
  "term_label": "damaged DNA binding",
  "term_id": "GO:0003684",
  "gene_name": "Replication protein A 70 kDa DNA-binding subunit",
  "gene": "UniProtKB:P27694",
  "gene_symbol": "RPA1"
}